{
  "gene_symbol": "CHRNB4",
  "term_label": "neuron projection",
  "gene_name": "Neuronal acetylcholine receptor subunit beta-4",
  "term_id": "GO:0043005",
  "gene": "UniProtKB:P30926"
}